{
  "gene_symbol": "IMPA2",
  "gene_name": "Inositol monophosphatase 2",
  "term_id": "GO:0008934",
  "gene": "UniProtKB:O14732",
  "term_label": "inositol monophosphate 1-phosphatase activity"
}